{
  "gene_name": "Protein bicaudal D homolog 1",
  "term_id": "GO:0045505",
  "term_label": "dynein intermediate chain binding",
  "gene_symbol": "BICD1",
  "gene": "UniProtKB:Q96G01"
}